{
  "gene": "UniProtKB:P49802",
  "term_id": "GO:0007186",
  "term_label": "G protein-coupled receptor signaling pathway",
  "gene_name": "Regulator of G-protein signaling 7",
  "gene_symbol": "RGS7"
}